alpha-pinene biosynthetic process [GO:0046248] (BP) Sources: GOC:ai Also known as: alpha-pinene anabolism, alpha-pinene biosynthesis, alpha-pinene formation, alpha-pinene synthesis Relationships: is a type of alpha-pinene metabolic process [GO:0018867]; is_a monoterpene biosynthetic process [GO:0043693] Definition: The chemical reactions and pathways resulting in the formation of alpha-pinene, a monoterpene that may be a significant factor affecting bacterial activities in nature.